{
  "term_id": "GO:0006357",
  "gene_symbol": "ZNF355P",
  "gene": "UniProtKB:Q9NSJ1",
  "gene_name": "Putative zinc finger protein 355P",
  "term_label": "regulation of transcription by RNA polymerase II"
}